{
  "gene": "UniProtKB:Q9Y3M8",
  "gene_symbol": "STARD13",
  "term_id": "GO:0005096",
  "term_label": "GTPase activator activity",
  "gene_name": "StAR-related lipid transfer protein 13"
}